histone H2AK5 acetyltransferase activity [GO:0043999] (molecular function) Note: Note that the residue position corresponds to the canonical human H2A2A histone (UniProtKB:Q6FI13); this residue is conserved across all eukaryotes. Corresponds to H2AK4 in yeast and in flies. Residue 1 is the first residue following removal of the initiating Methionine (Met). Note that each histone is encoded by multiple genes, and sequences may vary across different genes within an organism. References: PMID:18552846, PMID:19056256 Also known as: histone H2A-K5 acetyltransferase activity, histone acetylase activity (H2A-K5 specific), histone acetyltransferase activity (H2A-K5 specific), histone lysine N-acetyltransferase activity (H2A-K5 specific) Definition: Catalysis of the reaction: acetyl-CoA + histone H2A L-lysine (position 5) = CoA + histone H2A N6-acetyl-L-lysine (position 5). Relationships: is a type of histone H2A acetyltransferase activity [GO:0043998]